{
  "term_id": "GO:0007218",
  "gene": "UniProtKB:Q969F8",
  "term_label": "neuropeptide signaling pathway",
  "gene_name": "KiSS-1 receptor",
  "gene_symbol": "KISS1R"
}